{
  "term_id": "GO:0030036",
  "gene": "UniProtKB:Q9NR12",
  "gene_name": "PDZ and LIM domain protein 7",
  "term_label": "actin cytoskeleton organization",
  "gene_symbol": "PDLIM7"
}